{
  "term_label": "Unknown biological process",
  "gene_name": "Taste receptor type 2 member 19",
  "gene_symbol": "TAS2R19",
  "term_id": "UNKNOWN:0002",
  "gene": "UniProtKB:P59542"
}